GAA codon-amino acid adaptor activity [GO:0033459] (MF) Also known as: glutamic acid tRNA Definition: A triplet codon-amino acid adaptor activity that recognizes a GAA codon. Note: Note that in the standard genetic code, GAA codes for glutamic acid. Relationships: is_a triplet codon-amino acid adaptor activity [GO:0030533] Sources: GOC:mah